{
  "gene_name": "Olfactory receptor 8J2",
  "gene": "UniProtKB:Q8NGG1",
  "term_label": "Unknown cellular component",
  "gene_symbol": "OR8J2",
  "term_id": "UNKNOWN:0003"
}